{
  "gene_name": "Histone H1.2",
  "term_label": "chromosome condensation",
  "gene": "UniProtKB:P16403",
  "gene_symbol": "H1-2",
  "term_id": "GO:0030261"
}